{
  "term_id": "GO:0006196",
  "term_label": "AMP catabolic process",
  "gene_name": "5'-nucleotidase",
  "gene": "UniProtKB:P21589",
  "gene_symbol": "NT5E"
}